{
  "gene_symbol": "CSTB",
  "term_id": "GO:0005829",
  "gene_name": "Cystatin-B",
  "term_label": "cytosol",
  "gene": "UniProtKB:P04080"
}